{
  "term_id": "GO:0004930",
  "gene_symbol": "GPR65",
  "gene_name": "Psychosine receptor",
  "gene": "UniProtKB:Q8IYL9",
  "term_label": "G protein-coupled receptor activity"
}